{
  "gene_name": "Putative zinc finger protein 861",
  "gene": "UniProtKB:O60384",
  "term_id": "UNKNOWN:0001",
  "term_label": "Unknown molecular function",
  "gene_symbol": "ZNF861P"
}